{
  "term_id": "GO:0010494",
  "gene_symbol": "DDX19A",
  "gene_name": "ATP-dependent RNA helicase DDX19A",
  "gene": "UniProtKB:Q9NUU7",
  "term_label": "cytoplasmic stress granule"
}